mitochondrion to peroxisome vesicle-mediated transport [GO:0099076] (biological process) References: PMID:20619655 Sources: GOC:PARL-UCL, GOC:bc, GOC:pad Definition: Vesicle-mediated transport of cargo from the mitochondrion to the peroxisome, mediated by a mitochondrion-derived vesicle. Also known as: mitochondrion to peroxisome transport Relationships: is a type of mitochondrion-derived vesicle mediated transport [GO:0099075]